{
  "term_label": "DNA-binding transcription factor activity, RNA polymerase II-specific",
  "term_id": "GO:0000981",
  "gene_name": "Zinc finger protein 92 homolog",
  "gene_symbol": "ZFP92",
  "gene": "UniProtKB:A6NM28"
}